Atg12 conjugating enzyme activity [GO:0061651] (molecular function) Also known as: E2 Relationships: is a type of Atg12 transferase activity [GO:0019777]; is_a ubiquitin-like protein conjugating enzyme activity [GO:0061650] Sources: GOC:dph Definition: Isoenergetic transfer of Atg12 from one protein to another via the reaction X-Atg12 + Y = Y-Atg12 + X, where both the X-Atg12 and Y-Atg12 linkages are thioester bonds between the C-terminal amino acid of Atg12 and a sulfhydryl side group of a cysteine residue.